{
  "gene": "UniProtKB:Q13316",
  "gene_name": "Dentin matrix acidic phosphoprotein 1",
  "term_label": "extracellular matrix organization",
  "term_id": "GO:0030198",
  "gene_symbol": "DMP1"
}